negative regulation of lactation [GO:1903488] (biological process) Also known as: down regulation of lactation, down-regulation of lactation, downregulation of lactation, inhibition of lactation Relationships: is a type of negative regulation of secretion [GO:0051048]; is a type of GO:0051093; is_a negative regulation of multicellular organismal process [GO:0051241]; is a type of GO:1903487; negatively regulates lactation [GO:0007595] Definition: Any process that stops, prevents or reduces the frequency, rate or extent of lactation. References: PMID:19563620 Sources: GOC:TermGenie, GOC:mr, GO_REF:0000058